{
  "term_id": "GO:0051051",
  "gene_name": "PRA1 family protein 3",
  "gene_symbol": "ARL6IP5",
  "term_label": "negative regulation of transport",
  "gene": "UniProtKB:O75915"
}